{
  "gene_symbol": "ABLIM3",
  "gene": "UniProtKB:O94929",
  "gene_name": "Actin-binding LIM protein 3",
  "term_id": "GO:0015629",
  "term_label": "actin cytoskeleton"
}